{
  "gene_symbol": "PTPRM",
  "gene": "UniProtKB:P28827",
  "term_id": "GO:0004725",
  "gene_name": "Receptor-type tyrosine-protein phosphatase mu",
  "term_label": "protein tyrosine phosphatase activity"
}